{
  "term_label": "Unknown molecular function",
  "gene": "UniProtKB:O75901",
  "gene_symbol": "RASSF9",
  "gene_name": "Ras association domain-containing protein 9",
  "term_id": "UNKNOWN:0001"
}